swimming [GO:0036268] (biological process) Note: For behavioral aspects of swimming, consider instead annotating to 'swimming behavior ; GO:0036269'. Relationships: is a type of locomotion [GO:0040011] References: PMID:22459995 Sources: GOC:cvs Definition: Self-propelled movement of an organism from one location to another through water, often by means of active fin movement.